dorsal root ganglion morphogenesis [GO:1904835] (biological process) References: PMID:18936100 Sources: GOC:PARL, GOC:TermGenie, GOC:bf, GO_REF:0000083 Also known as: ganglion of dorsal root morphogenesis, ganglion spinalis morphogenesis, spinal ganglion morphogenesis, spinal ganglion part of peripheral nervous system morphogenesis, DRG morphogenesis, dorsal root ganglia morphogenesis, ganglion sensorium nervi spinalis morphogenesis, ganglion spinale morphogenesis, posterior root ganglion morphogenesis Definition: The developmental process by which a dorsal root ganglion is generated and organized. Relationships: is a type of GO:0061552; is part of GO:1990791